{
  "term_id": "GO:0006915",
  "gene_name": "Tumor necrosis factor receptor superfamily member 19L",
  "term_label": "apoptotic process",
  "gene": "UniProtKB:Q969Z4",
  "gene_symbol": "RELT"
}